adherens junction maintenance [GO:0034334] (biological process) Definition: The maintenance of an adherens junction. An adherens junction is a cell-cell junction composed of the epithelial cadherin-catenin complex at which the cytoplasmic face of the plasma membrane is attached to actin filaments. Sources: GOC:aruk, GOC:bc, GOC:mah Relationships: is a type of adherens junction organization [GO:0034332]; is a type of cell-cell junction maintenance [GO:0045217] Subtypes: GO:0045218